{
  "gene_symbol": "TMEM218",
  "term_id": "UNKNOWN:0002",
  "gene": "UniProtKB:A2RU14",
  "term_label": "Unknown biological process",
  "gene_name": "Transmembrane protein 218"
}